{
  "gene_symbol": "B4GALT1",
  "term_label": "protein N-linked glycosylation",
  "gene_name": "Beta-1,4-galactosyltransferase 1",
  "gene": "UniProtKB:P15291",
  "term_id": "GO:0006487"
}